positive regulation of axial mesodermal cell fate determination [GO:0048326] (biological process) Relationships: is a type of regulation of axial mesodermal cell fate determination [GO:0048324]; is a type of positive regulation of mesodermal cell fate determination [GO:0048336]; positively regulates axial mesodermal cell fate determination [GO:0048323] Also known as: up regulation of axial mesodermal cell fate determination, up-regulation of axial mesodermal cell fate determination, upregulation of axial mesodermal cell fate determination, activation of axial mesodermal cell fate determination, stimulation of axial mesodermal cell fate determination Sources: GOC:dgh Definition: Any process that activates or increases the frequency, rate or extent of axial mesoderm cell fate determination.